{
  "gene": "UniProtKB:Q9NY43",
  "gene_symbol": "BARHL2",
  "term_label": "DNA-binding transcription factor activity, RNA polymerase II-specific",
  "gene_name": "BarH-like 2 homeobox protein",
  "term_id": "GO:0000981"
}